maltose binding [GO:1901982] (molecular function) References: PMID:21566157 Sources: GOC:TermGenie Relationships: is a type of disaccharide binding [GO:0048030] Definition: Binding to maltose.